{
  "term_id": "UNKNOWN:0001",
  "term_label": "Unknown molecular function",
  "gene": "UniProtKB:Q9NVU0",
  "gene_symbol": "POLR3E",
  "gene_name": "DNA-directed RNA polymerase III subunit RPC5"
}